methylgalactoside transmembrane transporter activity [GO:0015592] (MF) Relationships: is a type of carbohydrate derivative transmembrane transporter activity [GO:1901505]; BFO_0000050 methylgalactoside transport [GO:0015765] Also known as: galactose/glucose (methylgalactoside) porter activity Definition: Enables the transfer of methylgalactoside from one side of a membrane to the other. Methylgalactoside is a compound in which the H of the OH group on carbon-1 of galactose is replaced by a methyl group. Sources: GOC:mtg_transport, ISBN:0815340729